cardiac muscle cell membrane repolarization [GO:0099622] (BP) Regulation: regulated by GO:0099623 Definition: The process in which ions are transported across the plasma membrane of a cardiac muscle cell such that the membrane potential changes in the repolarizing direction, toward the steady state potential. For example, the repolarization during an action potential is from a positive membrane potential towards a negative resting potential. Sources: GOC:BHF Relationships: is a type of membrane repolarization [GO:0086009] Subtypes: membrane repolarization during cardiac muscle cell action potential [GO:0086013], GO:0099624, ventricular cardiac muscle cell membrane repolarization [GO:0099625]